positive regulation of nucleotide-binding domain, leucine rich repeat containing receptor signaling pathway [GO:0070426] (BP) Subtypes: positive regulation of nucleotide-binding oligomerization domain containing 1 signaling pathway [GO:0070430], GO:0070434 Relationships: is_a GO:0062208; is a type of GO:0070424; is a type of positive regulation of intracellular signal transduction [GO:1902533]; positively regulates nucleotide-binding domain, leucine rich repeat containing receptor signaling pathway [GO:0035872] Also known as: positive regulation of NOD signaling pathway, positive regulation of nucleotide-binding oligomerization domain containing signaling pathway, positive regulation of nucleotide-binding oligomerization domain containing signalling pathway Sources: GOC:add Definition: Any process that activates or increases the frequency, rate, or extent of a nucleotide-binding domain, leucine rich repeat containing receptor signaling pathway (NLR) pathway.